{
  "term_id": "GO:0003779",
  "gene_name": "[F-actin]-monooxygenase MICAL3",
  "gene_symbol": "MICAL3",
  "term_label": "actin binding",
  "gene": "UniProtKB:Q7RTP6"
}